{
  "gene_symbol": "CCL25",
  "gene_name": "C-C motif chemokine 25",
  "term_label": "antimicrobial humoral immune response mediated by antimicrobial peptide",
  "gene": "UniProtKB:O15444",
  "term_id": "GO:0061844"
}